{
  "gene": "UniProtKB:Q86VW0",
  "term_label": "phosphatidylinositol-3,5-bisphosphate binding",
  "term_id": "GO:0080025",
  "gene_name": "SEC14 domain and spectrin repeat-containing protein 1",
  "gene_symbol": "SESTD1"
}